positive regulation of division septum assembly [GO:0010973] (biological process) Definition: Any process that increases the frequency, rate or extent of division septum formation. division septum formation is the assembly and arrangement of a septum that spans the plasma membrane interface between progeny cells following cytokinesis. References: PMID:19959363, PMID:21246752, PMID:22786806 Sources: GOC:mtg_cell_cycle Also known as: positive regulation of division septum formation, positive regulation of division septum formation involved in cell cycle cytokinesis, upregulation of mitotic division septum assembly Relationships: is a type of regulation of division septum assembly [GO:0032955]; is a type of GO:1901893; positively regulates division septum assembly [GO:0000917] Subtypes: positive regulation of septation initiation signaling [GO:0031031], positive regulation of mitotic division septum assembly [GO:0140281]